{
  "gene_symbol": "RSAD1",
  "term_label": "cytoplasm",
  "gene": "UniProtKB:Q9HA92",
  "term_id": "GO:0005737",
  "gene_name": "Radical S-adenosyl methionine domain-containing protein 1, mitochondrial"
}